{
  "gene": "UniProtKB:Q6NVU6",
  "term_label": "deUFMylase activity",
  "gene_symbol": "UFSP1",
  "term_id": "GO:0071567",
  "gene_name": "Inactive Ufm1-specific protease 1"
}